T cell activation via T cell receptor contact with antigen bound to MHC molecule on antigen presenting cell [GO:0002291] (BP) Definition: The change in morphology and behavior of a mature or immature T cell resulting from exposure to an antigen for which its T cell receptor is specific bound to an MHC molecule on an antigen presenting cell, leading to the initiation or perpetuation of an immune response. Sources: GOC:add, ISBN:0781735149 Also known as: T lymphocyte activation via T cell receptor contact with antigen bound to MHC molecule on antigen presenting cell, T-cell activation via T cell receptor contact with antigen bound to MHC molecule on antigen presenting cell, T-lymphocyte activation via T cell receptor contact with antigen bound to MHC molecule on antigen presenting cell Regulation: regulated by GO:2001188; RO_0002212 by GO:2001189; positively regulated by positive regulation of T cell activation via T cell receptor contact with antigen bound to MHC molecule on antigen presenting cell [GO:2001190] Relationships: is a type of T cell activation involved in immune response [GO:0002286]